{
  "gene_symbol": "TRPC7",
  "gene_name": "Short transient receptor potential channel 7",
  "gene": "UniProtKB:Q9HCX4",
  "term_id": "GO:0070588",
  "term_label": "calcium ion transmembrane transport"
}